mitochondrial membrane [GO:0031966] (cellular component) Relationships: is a type of organelle membrane [GO:0031090]; is part of GO:0005740 Subtypes: mitochondrial outer membrane [GO:0005741], mitochondrial inner membrane [GO:0005743] Sources: GOC:mah, NIF_Subcellular:sao1045389829 Definition: Either of the lipid bilayers that surround the mitochondrion and form the mitochondrial envelope.